negative regulation of retrograde trans-synaptic signaling by neuropeptide [GO:1905433] (biological process) Definition: Any process that stops, prevents or reduces the frequency, rate or extent of retrograde trans-synaptic signaling by neuropeptide. Also known as: down regulation of retrograde trans-synaptic signaling by neuropeptide, down-regulation of retrograde trans-synaptic signaling by neuropeptide, downregulation of retrograde trans-synaptic signaling by neuropeptide, inhibition of retrograde trans-synaptic signaling by neuropeptide, inhibition of neuropeptide-mediated retrograde trans-synaptic signaling, negative regulation of neuropeptide-mediated retrograde trans-synaptic signaling References: PMID:19448629 Sources: GOC:PARL, GOC:TermGenie, GOC:bf, GO_REF:0000058 Relationships: is a type of negative regulation of cell communication [GO:0010648]; is a type of negative regulation of signaling [GO:0023057]; is a type of regulation of retrograde trans-synaptic signaling by neuropeptide [GO:1905432]; RO_0002212 retrograde trans-synaptic signaling by neuropeptide [GO:0099082]